transcription elongation by RNA polymerase III [GO:0006385] (biological process) Also known as: RNA elongation from Pol III promoter, transcription elongation by RNA polymerase III promoter, transcription elongation from RNA polymerase III promoter, RNA polymerase III transcription elongation factor activity Sources: GOC:mah, GOC:txnOH Relationships: is a type of GO:0006354; is part of transcription by RNA polymerase III [GO:0006383] Definition: The extension of an RNA molecule after transcription initiation and promoter clearance at an RNA polymerase III promoter by the addition of ribonucleotides catalyzed by RNA polymerase III.